sedoheptulokinase activity [GO:0050277] (molecular function) Relationships: is a type of GO:0016301; is a type of phosphotransferase activity, alcohol group as acceptor [GO:0016773] Sources: EC:2.7.1.14, RHEA:23844 Also known as: ATP:sedoheptulose 7-phosphotransferase activity, heptulokinase activity, sedoheptulokinase (phosphorylating) Definition: Catalysis of the reaction: ATP + sedoheptulose = ADP + 2 H+ + sedoheptulose 7-phosphate.